structural constituent of presynaptic active zone [GO:0098882] (molecular function) Definition: The action of a molecule that contributes to the structural integrity of a presynaptic active zone. Sources: GOC:dos Relationships: is a type of structural constituent of synapse [GO:0098918]; is part of maintenance of presynaptic active zone structure [GO:0048790]; occurs in presynaptic active zone [GO:0048786] Also known as: structural constituent of active zone